negative regulation of macrophage colony-stimulating factor production [GO:1901257] (biological process) Definition: Any process that stops, prevents or reduces the frequency, rate or extent of macrophage colony-stimulating factor production. Also known as: down regulation of M-CSF production, down regulation of macrophage colony-stimulating factor production, down-regulation of M-CSF production, down-regulation of macrophage colony-stimulating factor production, downregulation of M-CSF production, downregulation of macrophage colony-stimulating factor production, inhibition of M-CSF production, negative regulation of M-CSF production, inhibition of macrophage colony-stimulating factor production Sources: GOC:BHF, GOC:TermGenie Relationships: is_a negative regulation of cytokine production [GO:0001818]; is a type of regulation of macrophage colony-stimulating factor production [GO:1901256]; negatively regulates GO:0036301 Subtypes: negative regulation of granulocyte colony-stimulating factor production [GO:0071656]